pore complex assembly [GO:0046931] (biological process) Sources: GOC:jl, GOC:mah Also known as: pore biosynthesis, pore formation, pore complex biogenesis, pore-forming toxin activity Note: See also the cellular component term 'pore complex ; GO:0046930'. Subtypes: nuclear pore complex assembly [GO:0051292] Definition: The aggregation, arrangement and bonding together of a set of components to form a pore complex. A pore complex is a small opening in a membrane that allows the passage of liquids and/or gases. Relationships: is a type of protein-containing complex assembly [GO:0065003]